regulation of endosperm development [GO:2000014] (biological process) Subtypes: negative regulation of endosperm development [GO:1904095] Definition: Any process that modulates the frequency, rate or extent of endosperm development. Sources: GOC:obol Relationships: is a type of regulation of developmental process [GO:0050793]; is a type of regulation of reproductive process [GO:2000241]; regulates endosperm development [GO:0009960]